{
  "gene": "UniProtKB:P30419",
  "gene_symbol": "NMT1",
  "term_label": "cytosol",
  "gene_name": "Glycylpeptide N-tetradecanoyltransferase 1",
  "term_id": "GO:0005829"
}